positive regulation of termination of RNA polymerase II transcription, poly(A)-coupled [GO:2000806] (biological process) Definition: Any process that activates or increases the frequency, rate or extent of termination of RNA polymerase II transcription, poly(A)-coupled. Also known as: positive regulation of termination of RNA polymerase II transcription, polyadenylation-coupled, positive regulation of transcription termination from Pol II promoter, RNA polymerase(A) coupled, positive regulation of transcription termination from Pol II promoter, poly(A) coupled Sources: GOC:obol Relationships: is a type of positive regulation of termination of RNA polymerase II transcription [GO:1904595]; is a type of GO:2000804; positively regulates termination of RNA polymerase II transcription, poly(A)-coupled [GO:0030846]